BID-BCL-xl complex [GO:1990346] (cellular component) Definition: A heterodimeric protein complex consisting of BID and BCL-xl, members of the Bcl-2 family of anti- and proapoptotic regulators. Relationships: is a type of protein-containing complex [GO:0032991] References: PMID:14634621 Sources: GOC:bhm